{
  "gene": "UniProtKB:O43248",
  "gene_symbol": "HOXC11",
  "term_label": "embryonic skeletal joint morphogenesis",
  "term_id": "GO:0060272",
  "gene_name": "Homeobox protein Hox-C11"
}